{
  "term_label": "plasma membrane",
  "gene": "UniProtKB:P0DPB3",
  "gene_symbol": "SCHIP1",
  "term_id": "GO:0005886",
  "gene_name": "Schwannomin-interacting protein 1"
}